{
  "gene": "UniProtKB:Q96L33",
  "term_id": "GO:0019901",
  "term_label": "protein kinase binding",
  "gene_symbol": "RHOV",
  "gene_name": "Rho-related GTP-binding protein RhoV"
}